{
  "term_label": "actin filament organization",
  "gene_name": "Ras-related C3 botulinum toxin substrate 1",
  "gene_symbol": "RAC1",
  "gene": "UniProtKB:P63000",
  "term_id": "GO:0007015"
}